{
  "term_label": "Golgi to lysosome transport",
  "gene": "UniProtKB:Q9P2R3",
  "gene_name": "Rabankyrin-5",
  "term_id": "GO:0090160",
  "gene_symbol": "ANKFY1"
}